{
  "term_id": "GO:0005829",
  "gene_name": "Thioredoxin-like protein 1",
  "gene": "UniProtKB:O43396",
  "gene_symbol": "TXNL1",
  "term_label": "cytosol"
}